{
  "gene_name": "Tau-tubulin kinase 2",
  "term_id": "GO:0005737",
  "gene": "UniProtKB:Q6IQ55",
  "gene_symbol": "TTBK2",
  "term_label": "cytoplasm"
}